{
  "gene": "UniProtKB:Q86UF2",
  "term_label": "protein secretion",
  "gene_name": "cTAGE family member 6",
  "gene_symbol": "CTAGE6",
  "term_id": "GO:0009306"
}